{
  "gene_name": "AP-5 complex subunit sigma-1",
  "gene_symbol": "AP5S1",
  "gene": "UniProtKB:Q9NUS5",
  "term_id": "UNKNOWN:0001",
  "term_label": "Unknown molecular function"
}